{
  "term_label": "cell adhesion molecule binding",
  "gene_name": "Protocadherin-12",
  "gene": "UniProtKB:Q9NPG4",
  "term_id": "GO:0050839",
  "gene_symbol": "PCDH12"
}